vascular endothelial cell response to oscillatory fluid shear stress [GO:0097706] (biological process) References: PMID:21768538 Sources: GOC:BHF, GOC:BHF_miRNA, GOC:bc Relationships: is a type of GO:0097699; is a type of cellular response to oscillatory fluid shear stress [GO:0097704] Also known as: blood vessel endothelial cell response to oscillatory fluid shear stress Definition: Any response to oscillatory fluid shear stress that occurs in a vascular endothelial cell.